{
  "term_id": "GO:0007605",
  "term_label": "sensory perception of sound",
  "gene_symbol": "LOXHD1",
  "gene_name": "Lipoxygenase homology domain-containing protein 1",
  "gene": "UniProtKB:Q8IVV2"
}